{
  "gene": "UniProtKB:Q8N2Z9",
  "term_id": "GO:0003682",
  "gene_name": "Centromere protein S",
  "term_label": "chromatin binding",
  "gene_symbol": "CENPS"
}